{
  "gene_name": "Mitogen-activated protein kinase kinase kinase 5",
  "gene": "UniProtKB:Q99683",
  "gene_symbol": "MAP3K5",
  "term_label": "p38MAPK cascade",
  "term_id": "GO:0038066"
}